telethonin binding [GO:0031433] (molecular function) Relationships: is a type of cytoskeletal protein binding [GO:0008092] References: PMID:10481174 Sources: GOC:mah Definition: Binding to telethonin, a protein found in the Z disc of striated muscle and which is a substrate of the titin kinase.